negative regulation of beta 2 integrin biosynthetic process [GO:0045774] (biological process) Relationships: is a type of regulation of beta 2 integrin biosynthetic process [GO:0045115]; is_a negative regulation of integrin biosynthetic process [GO:0045720]; negatively regulates beta 2 integrin biosynthetic process [GO:0045114] Sources: GOC:go_curators Definition: Any process that stops, prevents, or reduces the frequency, rate or extent of the chemical reactions and pathways resulting in the formation of beta 2 integrins. Also known as: down regulation of beta 2 integrin biosynthetic process, down-regulation of beta 2 integrin biosynthetic process, downregulation of beta 2 integrin biosynthetic process, negative regulation of beta 2 integrin anabolism, negative regulation of beta 2 integrin biosynthesis, negative regulation of beta 2 integrin formation, negative regulation of beta 2 integrin synthesis, inhibition of beta 2 integrin biosynthetic process